{
  "gene_name": "Tubulin polymerization-promoting protein family member 3",
  "gene_symbol": "TPPP3",
  "term_id": "GO:0046785",
  "term_label": "microtubule polymerization",
  "gene": "UniProtKB:Q9BW30"
}